{
  "gene": "UniProtKB:O75521",
  "gene_symbol": "ECI2",
  "term_label": "delta(3)-delta(2)-enoyl-CoA isomerase activity",
  "gene_name": "Enoyl-CoA delta isomerase 2",
  "term_id": "GO:0004165"
}